{
  "term_id": "GO:0008063",
  "gene_name": "Paralemmin-3",
  "gene": "UniProtKB:A6NDB9",
  "term_label": "Toll signaling pathway",
  "gene_symbol": "PALM3"
}